{
  "term_label": "plasma membrane",
  "gene_name": "Ly6_PLAUR domain-containing protein 3",
  "gene_symbol": "LYPD3",
  "term_id": "GO:0005886",
  "gene": "UniProtKB:O95274"
}